{
  "term_id": "GO:0019310",
  "gene_name": "Inositol oxygenase",
  "gene_symbol": "MIOX",
  "gene": "UniProtKB:Q9UGB7",
  "term_label": "inositol catabolic process"
}